{
  "term_label": "Unknown molecular function",
  "term_id": "UNKNOWN:0001",
  "gene_symbol": "SPIN3",
  "gene": "UniProtKB:Q5JUX0",
  "gene_name": "Spindlin-3"
}